respiratory chain complex II assembly [GO:0034552] (biological process) Relationships: is a type of protein-containing complex assembly [GO:0065003] Subtypes: GO:0034553 Sources: GOC:dgf Definition: The aggregation, arrangement and bonding together of a set of components to form respiratory chain complex II.